{
  "gene_name": "U6 snRNA-associated Sm-like protein LSm2",
  "term_id": "GO:0000932",
  "gene_symbol": "LSM2",
  "gene": "UniProtKB:Q9Y333",
  "term_label": "P-body"
}